{
  "gene_name": "Serine_arginine repetitive matrix protein 5",
  "term_label": "Unknown biological process",
  "gene_symbol": "SRRM5",
  "gene": "UniProtKB:B3KS81",
  "term_id": "UNKNOWN:0002"
}